mitotic nuclear bridge midzone membrane domain [GO:0140599] (cellular component) Definition: A nuclear membrane part at the midzone of the mitotic nuclear bridge. The midzone forms a bulge that is enriched in nuclear pores that lack baskets. Relationships: is a type of cellular anatomical structure [GO:0110165]; is part of mitotic nuclear bridge midzone [GO:0140512] References: PMID:25963819, PMID:32502403